{
  "gene_name": "Adhesion G protein-coupled receptor F5",
  "gene": "UniProtKB:Q8IZF2",
  "term_id": "GO:0005886",
  "term_label": "plasma membrane",
  "gene_symbol": "ADGRF5"
}